{
  "gene_name": "Shieldin complex subunit 2",
  "gene_symbol": "SHLD2",
  "term_label": "Unknown molecular function",
  "term_id": "UNKNOWN:0001",
  "gene": "UniProtKB:Q86V20"
}